neutral L-amino acid:sodium symporter activity [GO:0005295] (molecular function) Sources: TC:2.A.23.3.1 Definition: Enables the transfer of a solute or solutes from one side of a membrane to the other according to the reaction: neutral L-amino acid(out) + Na+(out) = neutral L-amino acid(in) + Na+(in). Also known as: neutral amino acid-sodium cotransporter, sodium/neutral amino acid transporter, neutral amino acid:sodium symporter activity Relationships: is_a amino acid:sodium symporter activity [GO:0005283]; is a type of neutral L-amino acid transmembrane transporter activity [GO:0015175] Subtypes: glycine:sodium symporter activity [GO:0015375], L-asparagine:sodium symporter activity [GO:0140901], L-glutamine:sodium symporter activity [GO:0140902]